{
  "term_id": "GO:0003735",
  "gene_symbol": "RPL10L",
  "gene": "UniProtKB:Q96L21",
  "gene_name": "Ribosomal protein uL16-like",
  "term_label": "structural constituent of ribosome"
}